ankyrin repeat binding [GO:0071532] (MF) Sources: GOC:mah, InterPro:IPR002110 Also known as: ANK repeat binding Relationships: is a type of protein domain specific binding [GO:0019904] Definition: Binding to an ankyrin repeat of a protein. Ankyrin repeats are tandemly repeated modules of about 33 amino acids; each repeat folds into a helix-loop-helix structure with a beta-hairpin/loop region projecting out from the helices at a 90-degree angle, and repeats stack to form an L-shaped structure.